{
  "gene": "UniProtKB:Q8N114",
  "term_label": "Unknown biological process",
  "term_id": "UNKNOWN:0002",
  "gene_symbol": "SHISA5",
  "gene_name": "Protein shisa-5"
}